P-element binding [GO:0003693] (molecular function) Relationships: is a type of sequence-specific double-stranded DNA binding [GO:1990837] Definition: Binding to a P-element, a class of Drosophila transposon responsible for hybrid dysgenesis. References: PMID:9440262 Sources: GOC:jl